nuclear cap binding complex [GO:0005846] (cellular component) Also known as: nuclear CBC, NCBP-NIP1 complex, mRNA cap binding complex, snRNA cap binding complex, CBC Note: Note that this complex can be found in the cytoplasm as well as the nucleus. Definition: A conserved heterodimeric protein complex that binds to the 5' terminal cap structure m7G(5')ppp(5')N of nascent eukaryotic RNA polymerase II transcripts such as pre-mRNA and U snRNA. The consists of proteins known as CBP20 and CBP80, binds to cap structures in the nucleus, and is involved in pre-mRNA splicing, 3'-end formation, and RNA nuclear export. References: PMID:16043498 Relationships: is a type of GO:0034518